{
  "gene_symbol": "OR2T2",
  "term_id": "GO:0004984",
  "term_label": "olfactory receptor activity",
  "gene": "UniProtKB:Q6IF00",
  "gene_name": "Olfactory receptor 2T2"
}